{
  "gene_name": "Tropomodulin-2",
  "term_label": "tropomyosin binding",
  "gene_symbol": "TMOD2",
  "term_id": "GO:0005523",
  "gene": "UniProtKB:Q9NZR1"
}